{
  "gene": "UniProtKB:Q9BXU2",
  "gene_symbol": "TEX13B",
  "gene_name": "Testis-expressed protein 13B",
  "term_id": "UNKNOWN:0002",
  "term_label": "Unknown biological process"
}